regulation of muscle cell chemotaxis toward tendon cell [GO:2001281] (biological process) Relationships: is a type of regulation of cell migration [GO:0030334]; is a type of regulation of chemotaxis [GO:0050920]; regulates GO:0036061 Also known as: regulation of muscle cell chemotaxis towards tendon cell, regulation of muscle cell attraction Sources: GOC:sart Definition: Any process that modulates the frequency, rate or extent of muscle cell chemotaxis toward tendon cell. Subtypes: negative regulation of muscle cell chemotaxis toward tendon cell [GO:2001282]